negative regulation of organic acid transport [GO:0032891] (BP) Subtypes: GO:0002037, negative regulation of glutamate secretion [GO:0014050], negative regulation of gamma-aminobutyric acid secretion [GO:0014053], negative regulation of gluconate transmembrane transport [GO:0035431], GO:0051949, negative regulation of bile acid secretion [GO:0120190], GO:0140216, GO:1900924, GO:1900927, negative regulation of L-tyrosine import across plasma membrane [GO:1900930], GO:1902835, GO:1904449, negative regulation of glycine secretion, neurotransmission [GO:1904625], negative regulation of L-lysine import across plasma membrane [GO:1905009], GO:1905533, negative regulation of L-arginine import across plasma membrane [GO:1905542], negative regulation of L-methionine import across plasma membrane [GO:1905625], GO:2000192, negative regulation of glutamine transport [GO:2000486] Relationships: is a type of regulation of organic acid transport [GO:0032890]; is a type of GO:0051051; negatively regulates organic acid transport [GO:0015849] Sources: GOC:mah Definition: Any process that stops, prevents, or reduces the frequency, rate or extent of the directed movement of organic acids into, out of or within a cell, or between cells, by means of some agent such as a transporter or pore. Also known as: down regulation of organic acid transport, down-regulation of organic acid transport, downregulation of organic acid transport, inhibition of organic acid transport